{
  "term_id": "GO:0005794",
  "gene_symbol": "NDST3",
  "gene_name": "Bifunctional heparan sulfate N-deacetylase_N-sulfotransferase 3",
  "gene": "UniProtKB:O95803",
  "term_label": "Golgi apparatus"
}